alpha-agarase activity [GO:0033953] (molecular function) Sources: EC:3.2.1.158 Also known as: agarase activity, agarose 3-glycanohydrolase activity, agarase A33 activity Relationships: is a type of hydrolase activity, hydrolyzing O-glycosyl compounds [GO:0004553] Definition: Catalysis of the endohydrolysis of 1,3-alpha-L-galactosidic linkages in agarose, yielding agarotetraose as the major product.